{
  "gene_name": "Vascular endothelial growth factor C",
  "term_id": "GO:0001666",
  "term_label": "response to hypoxia",
  "gene_symbol": "VEGFC",
  "gene": "UniProtKB:P49767"
}